response to X-ray [GO:0010165] (biological process) Definition: Any process that results in a change in state or activity of a cell or an organism (in terms of movement, secretion, enzyme production, gene expression, etc.) as a result of X-ray radiation. An X-ray is a form of electromagnetic radiation with a wavelength in the range of 10 nanometers to 100 picometers (corresponding to frequencies in the range 30 PHz to 3 EHz). Also known as: response to X-ray radiation stimulus Relationships: is a type of response to ionizing radiation [GO:0010212] Subtypes: cellular response to X-ray [GO:0071481] Sources: GOC:sm, Wikipedia:X-ray